{
  "term_label": "positive regulation of cell population proliferation",
  "term_id": "GO:0008284",
  "gene_name": "Lithostathine-1-alpha",
  "gene": "UniProtKB:P05451",
  "gene_symbol": "REG1A"
}